{
  "gene_symbol": "TMEM214",
  "term_label": "Golgi apparatus",
  "gene_name": "Transmembrane protein 214",
  "term_id": "GO:0005794",
  "gene": "UniProtKB:Q6NUQ4"
}